{
  "term_id": "GO:0005634",
  "gene_symbol": "ZNF782",
  "term_label": "nucleus",
  "gene": "UniProtKB:Q6ZMW2",
  "gene_name": "Zinc finger protein 782"
}